{
  "term_id": "GO:0005886",
  "gene_name": "Sodium_hydrogen exchanger 11",
  "gene": "UniProtKB:Q5TAH2",
  "term_label": "plasma membrane",
  "gene_symbol": "SLC9C2"
}